{
  "gene": "UniProtKB:Q9UIW0",
  "term_label": "nucleus",
  "term_id": "GO:0005634",
  "gene_name": "Ventral anterior homeobox 2",
  "gene_symbol": "VAX2"
}